{
  "gene": "UniProtKB:Q6UXN7",
  "term_label": "tRNA import into mitochondrion",
  "term_id": "GO:0016031",
  "gene_symbol": "TOMM20L",
  "gene_name": "TOMM20-like protein 1"
}